endothelial cell apoptotic process [GO:0072577] (biological process) Regulation: regulated by GO:2000351; negatively regulated by GO:2000352; positively regulated by positive regulation of endothelial cell apoptotic process [GO:2000353] Definition: Any apoptotic process in an endothelial cell. An endothelial cell comprises the outermost layer or lining of anatomical structures and can be squamous or cuboidal. Relationships: is a type of apoptotic process [GO:0006915] Also known as: apoptosis of endothelial cells, endothelial cell programmed cell death by apoptosis, killing of endothelial cells, programmed cell death of endothelial cells by apoptosis, programmed cell death, endothelial cells, endothelial cell apoptosis Sources: CL:0000115, GOC:BHF, GOC:mah, GOC:mtg_apoptosis